{
  "term_label": "intermediate filament organization",
  "term_id": "GO:0045109",
  "gene_name": "Keratin, type I cytoskeletal 23",
  "gene": "UniProtKB:Q9C075",
  "gene_symbol": "KRT23"
}